{
  "gene": "UniProtKB:O43148",
  "gene_symbol": "RNMT",
  "gene_name": "mRNA cap guanine-N7 methyltransferase",
  "term_id": "GO:0006370",
  "term_label": "7-methylguanosine mRNA capping"
}